{
  "term_id": "GO:0060070",
  "gene": "UniProtKB:Q9ULW2",
  "gene_name": "Frizzled-10",
  "term_label": "canonical Wnt signaling pathway",
  "gene_symbol": "FZD10"
}